{
  "gene_name": "Prostaglandin E synthase 3",
  "term_label": "protein folding",
  "gene_symbol": "PTGES3",
  "term_id": "GO:0006457",
  "gene": "UniProtKB:Q15185"
}